{
  "term_id": "GO:0030017",
  "gene_symbol": "ABRA",
  "term_label": "sarcomere",
  "gene_name": "Actin-binding Rho-activating protein",
  "gene": "UniProtKB:Q8N0Z2"
}